{
  "gene_name": "Spermine oxidase",
  "gene_symbol": "SMOX",
  "term_id": "GO:0046592",
  "term_label": "polyamine oxidase activity",
  "gene": "UniProtKB:Q9NWM0"
}